Wnt signaling pathway, calcium modulating pathway [GO:0007223] (biological process) References: PMID:11532397, PMID:37804416 Definition: A type of non-canonical Wnt signaling in which Wnt binding to its receptor on the surface of a target cell leads to an increase in intracellular calcium and activation of protein kinase C (PKC). Regulation: regulated by regulation of Wnt signaling pathway, calcium modulating pathway [GO:0008591]; negatively regulated by negative regulation of Wnt signaling pathway, calcium modulating pathway [GO:0045812]; positively regulated by positive regulation of Wnt signaling pathway, calcium modulating pathway [GO:0045813] Also known as: non-canonical Wnt signaling pathway, Wnt receptor signaling pathway, calcium modulating pathway, Wnt-activated signaling pathway, calcium modulating pathway, frizzled-2 signaling pathway, frizzled-2 signalling pathway Relationships: is a type of non-canonical Wnt signaling pathway [GO:0035567]